regulation of tRNA processing [GO:2000235] (biological process) Definition: Any process that modulates the frequency, rate or extent of tRNA processing. Subtypes: regulation of tRNA methylation [GO:0110002], negative regulation of tRNA processing [GO:2000236], positive regulation of tRNA processing [GO:2000237] Sources: GOC:mah Also known as: regulation of tRNA maturation Relationships: is a type of regulation of gene expression [GO:0010468]; is a type of GO:1903326; regulates tRNA processing [GO:0008033]